positive regulation of dipeptide transport [GO:2000880] (biological process) Sources: GOC:obol Relationships: is a type of regulation of dipeptide transport [GO:0090089]; is a type of positive regulation of oligopeptide transport [GO:2000878]; positively regulates dipeptide transport [GO:0042938] Subtypes: GO:2001150 Definition: Any process that activates or increases the frequency, rate or extent of dipeptide transport.